{
  "gene_name": "TAF5-like RNA polymerase II p300_CBP-associated factor-associated factor 65 kDa subunit 5L",
  "gene": "UniProtKB:O75529",
  "term_label": "transcription factor TFTC complex",
  "term_id": "GO:0033276",
  "gene_symbol": "TAF5L"
}